negative regulation of lateral mesodermal cell fate specification [GO:0048380] (biological process) Relationships: is a type of negative regulation of mesodermal cell fate specification [GO:0042662]; is a type of regulation of lateral mesodermal cell fate specification [GO:0048378]; RO_0002212 GO:0048377 Sources: GOC:jid Also known as: down regulation of lateral mesodermal cell fate specification, down-regulation of lateral mesodermal cell fate specification, downregulation of lateral mesodermal cell fate specification, negative regulation of lateral plate mesodermal cell fate specification, inhibition of lateral mesodermal cell fate specification Definition: Any process that stops, prevents, or reduces the frequency, rate or extent of lateral mesoderm cell fate specification.